{
  "gene_name": "ADP-ribosylation factor-like protein 4D",
  "gene_symbol": "ARL4D",
  "gene": "UniProtKB:P49703",
  "term_label": "intracellular protein transport",
  "term_id": "GO:0006886"
}